{
  "gene": "UniProtKB:Q9GZZ6",
  "gene_name": "Neuronal acetylcholine receptor subunit alpha-10",
  "term_id": "GO:1904315",
  "term_label": "transmitter-gated monoatomic ion channel activity involved in regulation of postsynaptic membrane potential",
  "gene_symbol": "CHRNA10"
}